{
  "gene_symbol": "APOBEC2",
  "term_id": "GO:0004126",
  "gene_name": "C-U-editing enzyme APOBEC-2",
  "term_label": "cytidine deaminase activity",
  "gene": "UniProtKB:Q9Y235"
}